{
  "gene_name": "Myoneurin",
  "gene": "UniProtKB:Q9NPC7",
  "term_id": "GO:0006357",
  "term_label": "regulation of transcription by RNA polymerase II",
  "gene_symbol": "MYNN"
}